{
  "gene_symbol": "LVRN",
  "term_label": "extracellular space",
  "gene_name": "Aminopeptidase Q",
  "gene": "UniProtKB:Q6Q4G3",
  "term_id": "GO:0005615"
}